{
  "gene": "UniProtKB:Q9H492",
  "term_id": "GO:0008429",
  "term_label": "phosphatidylethanolamine binding",
  "gene_name": "Microtubule-associated proteins 1A_1B light chain 3A",
  "gene_symbol": "MAP1LC3A"
}